{
  "term_id": "GO:0005930",
  "gene_name": "Coiled-coil domain-containing protein 113",
  "term_label": "axoneme",
  "gene": "UniProtKB:Q9H0I3",
  "gene_symbol": "CCDC113"
}